{
  "term_label": "DNA-binding transcription activator activity, RNA polymerase II-specific",
  "gene_symbol": "ALX1",
  "term_id": "GO:0001228",
  "gene": "UniProtKB:Q15699",
  "gene_name": "ALX homeobox protein 1"
}